{
  "gene_name": "Alpha-N-acetylgalactosaminide alpha-2,6-sialyltransferase 5",
  "gene": "UniProtKB:Q9BVH7",
  "term_label": "ganglioside biosynthetic process",
  "term_id": "GO:0001574",
  "gene_symbol": "ST6GALNAC5"
}